{
  "term_id": "GO:0005890",
  "gene_symbol": "ATP1A1",
  "term_label": "sodium:potassium-exchanging ATPase complex",
  "gene": "UniProtKB:P05023",
  "gene_name": "Sodium_potassium-transporting ATPase subunit alpha-1"
}